{
  "gene_name": "Spermatogenesis-associated protein 31D3",
  "gene": "UniProtKB:P0C874",
  "gene_symbol": "SPATA31D3",
  "term_label": "Unknown molecular function",
  "term_id": "UNKNOWN:0001"
}